{
  "gene": "UniProtKB:P17535",
  "term_id": "GO:0045944",
  "gene_name": "Transcription factor JunD",
  "gene_symbol": "JUND",
  "term_label": "positive regulation of transcription by RNA polymerase II"
}